{
  "gene": "UniProtKB:Q99538",
  "term_label": "Unknown cellular component",
  "term_id": "UNKNOWN:0003",
  "gene_name": "Legumain",
  "gene_symbol": "LGMN"
}